{
  "term_label": "histone H3K9 deacetylase activity, NAD-dependent",
  "gene": "UniProtKB:Q8N6T7",
  "term_id": "GO:0046969",
  "gene_name": "NAD-dependent protein deacylase sirtuin-6",
  "gene_symbol": "SIRT6"
}